{
  "term_id": "UNKNOWN:0001",
  "gene_symbol": "IRGQ",
  "gene": "UniProtKB:Q8WZA9",
  "term_label": "Unknown molecular function",
  "gene_name": "Immunity-related GTPase family Q protein"
}